{
  "gene": "UniProtKB:O14569",
  "gene_name": "Transmembrane reductase CYB561D2",
  "term_id": "GO:0140576",
  "gene_symbol": "CYB561D2",
  "term_label": "ascorbate homeostasis"
}